negative regulation of ceramide biosynthetic process [GO:1900060] (BP) Definition: Any process that stops, prevents or reduces the frequency, rate or extent of a ceramide biosynthetic process. Relationships: is a type of negative regulation of amide metabolic process [GO:0034249]; is a type of GO:0090155; is a type of regulation of ceramide biosynthetic process [GO:2000303]; negatively regulates ceramide biosynthetic process [GO:0046513] References: PMID:15302821 Sources: GOC:TermGenie Subtypes: negative regulation of glucosylceramide biosynthetic process [GO:0046318] Also known as: down regulation of ceramide anabolism, down regulation of ceramide biosynthesis, down regulation of ceramide formation, down regulation of ceramide synthesis, down-regulation of ceramide anabolism, down-regulation of ceramide biosynthesis, down-regulation of ceramide formation, down-regulation of ceramide synthesis, downregulation of ceramide anabolism, downregulation of ceramide biosynthesis, downregulation of ceramide formation, downregulation of ceramide synthesis, inhibition of ceramide anabolism, inhibition of ceramide biosynthesis, inhibition of ceramide formation, inhibition of ceramide synthesis, negative regulation of ceramide anabolism, negative regulation of ceramide biosynthesis, negative regulation of ceramide formation, negative regulation of ceramide synthesis, down regulation of ceramide biosynthetic process, down-regulation of ceramide biosynthetic process, downregulation of ceramide biosynthetic process, inhibition of ceramide biosynthetic process